{
  "term_id": "UNKNOWN:0001",
  "gene_name": "Putative high mobility group protein B1-like 1",
  "term_label": "Unknown molecular function",
  "gene": "UniProtKB:B2RPK0",
  "gene_symbol": "HMGB1P1"
}